chloroplast RNA modification [GO:1900865] (biological process) Subtypes: chloroplast mRNA modification [GO:1900871] Sources: GOC:TermGenie Also known as: RNA editing in chloroplast Definition: Any RNA modification that takes place in chloroplast. Relationships: is a type of RNA modification [GO:0009451]; occurs in GO:0009507